{
  "gene": "UniProtKB:Q9BY43",
  "term_label": "multivesicular body",
  "term_id": "GO:0005771",
  "gene_symbol": "CHMP4A",
  "gene_name": "Charged multivesicular body protein 4a"
}